cellular hypotonic salinity response [GO:0071477] (biological process) Relationships: is a type of hypotonic salinity response [GO:0042539]; is a type of cellular response to salt stress [GO:0071472]; is a type of cellular hypotonic response [GO:0071476] Sources: GOC:mah Also known as: cellular response to hypotonic salt stress Definition: Any process that results in a change in state or activity of a cell (in terms of movement, secretion, enzyme production, gene expression, etc.) as a result of detection of, or exposure to, a decrease in the concentration of salt (particularly but not exclusively sodium and chloride ions) in the environment.